outer dense fiber [GO:0001520] (cellular component) Also known as: outer dense fibre Relationships: is_a GO:0099513; is part of sperm flagellum [GO:0036126] Definition: A supramolecular fiber found in the flagella of mammalian sperm that surrounds the nine microtubule doublets. These dense fibers are stiff and noncontractile. In human, they consist of about 10 major and at least 15 minor proteins, where all major proteins are ODF1, ODF2 or ODF2-related proteins. References: PMID:10381817, PMID:21586547, PMID:25361759 Sources: GOC:cilia, GOC:krc, ISBN:0824072820